{
  "term_label": "RNA polymerase II cis-regulatory region sequence-specific DNA binding",
  "term_id": "GO:0000978",
  "gene": "UniProtKB:P35712",
  "gene_name": "Transcription factor SOX-6",
  "gene_symbol": "SOX6"
}